{
  "gene_name": "RNA-binding protein Nova-1",
  "gene": "UniProtKB:P51513",
  "gene_symbol": "NOVA1",
  "term_id": "GO:0007399",
  "term_label": "nervous system development"
}